{
  "gene_name": "Sperm-associated antigen 4 protein",
  "term_label": "Unknown biological process",
  "gene": "UniProtKB:Q9NPE6",
  "gene_symbol": "SPAG4",
  "term_id": "UNKNOWN:0002"
}